{
  "term_label": "nucleus",
  "term_id": "GO:0005634",
  "gene_symbol": "CDC25A",
  "gene_name": "M-phase inducer phosphatase 1",
  "gene": "UniProtKB:P30304"
}